{
  "gene_name": "Poly(rC)-binding protein 4",
  "gene": "UniProtKB:P57723",
  "term_label": "cytoplasm",
  "gene_symbol": "PCBP4",
  "term_id": "GO:0005737"
}